{
  "gene": "UniProtKB:Q8NFG4",
  "gene_name": "Folliculin",
  "gene_symbol": "FLCN",
  "term_label": "positive regulation of TORC1 signaling",
  "term_id": "GO:1904263"
}